{
  "gene": "UniProtKB:Q15431",
  "term_id": "GO:0051026",
  "gene_name": "Synaptonemal complex protein 1",
  "gene_symbol": "SYCP1",
  "term_label": "chiasma assembly"
}